{
  "gene": "UniProtKB:Q8TDQ1",
  "gene_name": "CMRF35-like molecule 1",
  "gene_symbol": "CD300LF",
  "term_label": "transmembrane signaling receptor activity",
  "term_id": "GO:0004888"
}